{
  "gene_symbol": "LILRA2",
  "term_label": "inhibitory MHC class I receptor activity",
  "gene_name": "Leukocyte immunoglobulin-like receptor subfamily A member 2",
  "term_id": "GO:0032396",
  "gene": "UniProtKB:Q8N149"
}